{
  "gene_name": "Sodium_hydrogen exchanger 5",
  "gene_symbol": "SLC9A5",
  "term_label": "regulation of intracellular pH",
  "gene": "UniProtKB:Q14940",
  "term_id": "GO:0051453"
}